{
  "term_label": "brain development",
  "term_id": "GO:0007420",
  "gene": "UniProtKB:P35716",
  "gene_name": "Transcription factor SOX-11",
  "gene_symbol": "SOX11"
}